pyrrole-2-carboxylate decarboxylase activity [GO:0034941] (molecular function) Definition: Catalysis of the reaction: pryrole-2-carboxylate + H+ = pyrrole + CO2. Relationships: is a type of carboxy-lyase activity [GO:0016831] Sources: UM-BBD_reactionID:r0970